{
  "gene": "UniProtKB:P50221",
  "gene_symbol": "MEOX1",
  "term_label": "DNA-binding transcription factor activity, RNA polymerase II-specific",
  "gene_name": "Homeobox protein MOX-1",
  "term_id": "GO:0000981"
}